{
  "term_label": "regulation of Notch signaling pathway",
  "term_id": "GO:0008593",
  "gene_name": "Beta-1,3-N-acetylglucosaminyltransferase radical fringe",
  "gene": "UniProtKB:Q9Y644",
  "gene_symbol": "RFNG"
}